{
  "gene_symbol": "COX15",
  "gene_name": "Cytochrome c oxidase assembly protein COX15 homolog",
  "gene": "UniProtKB:Q7KZN9",
  "term_id": "GO:0005743",
  "term_label": "mitochondrial inner membrane"
}